{
  "gene_symbol": "H2AB3",
  "gene_name": "Histone H2A-Bbd type 2_3",
  "term_id": "GO:0000786",
  "gene": "UniProtKB:P0C5Z0",
  "term_label": "nucleosome"
}